midbrain dopaminergic neuron differentiation [GO:1904948] (biological process) Regulation: regulated by GO:1904956; negatively regulated by GO:1904957; positively regulated by positive regulation of midbrain dopaminergic neuron differentiation [GO:1904958] Relationships: is a type of GO:0021953; is a type of GO:0071542; is part of midbrain development [GO:0030901] Also known as: DA neurogenesis from midbrain floor plate, mDA neuron differentiation, midbrain DA neurogenesis, midbrain dopaminergic neuron production Definition: The process in which a relatively unspecialized cell acquires the specialized features of a midbrain dopaminergic neuron. References: PMID:17331494, PMID:19122665 Sources: GOC:PARL, GOC:TermGenie, GOC:bf, GO_REF:0000086